regulation of mitotic spindle formation (spindle phase one) [GO:0110159] (biological process) Relationships: is a type of regulation of mitotic spindle assembly [GO:1901673]; is part of regulation of mitotic spindle elongation [GO:0032888]; regulates mitotic spindle formation (spindle phase one) [GO:0061804] References: PMID:27697865 Sources: GOC:vw Subtypes: negative regulation of mitotic spindle formation (spindle phase one) [GO:0110160], positive regulation of mitotic spindle formation (spindle phase one) [GO:0110161] Definition: Any process that modulates the frequency, rate or extent of the cell cycle process in which the distance is lengthened between poles of the mitotic spindle during mitotic prophase (spindle phase one).